{
  "gene_name": "Membrane-bound transcription factor site-2 protease",
  "gene_symbol": "MBTPS2",
  "term_label": "cytoplasm",
  "gene": "UniProtKB:O43462",
  "term_id": "GO:0005737"
}